regulation of carbohydrate catabolic process [GO:0043470] (biological process) Sources: GOC:mlg Definition: Any process that modulates the frequency, rate, or extent of the chemical reactions and pathways resulting in the breakdown of carbohydrates. Relationships: is a type of GO:0006109; is_a regulation of catabolic process [GO:0009894]; regulates carbohydrate catabolic process [GO:0016052] Subtypes: GO:0005981, regulation of glycolytic process [GO:0006110], regulation of pentose-phosphate shunt [GO:0043456], regulation of rhamnose catabolic process [GO:0043463], regulation of fucose catabolic process [GO:0043468], GO:0043469, regulation of cellobiose catabolic process [GO:1900282], positive regulation of trehalose catabolic process [GO:1901319], regulation of glucose catabolic process to lactate via pyruvate [GO:1904023], regulation of starch catabolic process [GO:2000881], regulation of glucomannan catabolic process [GO:2000898], GO:2000912, GO:2000927, regulation of cellotriose catabolic process [GO:2000936], regulation of cyclodextrin catabolic process [GO:2000957], GO:2000963, GO:2000966, regulation of hemicellulose catabolic process [GO:2000988], regulation of galactomannan catabolic process [GO:2000991], regulation of cellulose catabolic process [GO:2000997], regulation of pectin catabolic process [GO:2001003], regulation of glycolytic fermentation to ethanol [GO:2001154]